{
  "term_label": "extracellular region",
  "gene_symbol": "SPINK14",
  "gene": "UniProtKB:Q6IE38",
  "term_id": "GO:0005576",
  "gene_name": "Serine protease inhibitor Kazal-type 14"
}